{
  "gene": "UniProtKB:P01569",
  "gene_symbol": "IFNA5",
  "term_id": "GO:0005125",
  "term_label": "cytokine activity",
  "gene_name": "Interferon alpha-5"
}